{
  "gene_symbol": "UBQLN1",
  "term_id": "GO:0006511",
  "gene": "UniProtKB:Q9UMX0",
  "term_label": "ubiquitin-dependent protein catabolic process",
  "gene_name": "Ubiquilin-1"
}